{
  "gene_symbol": "SH3BGRL2",
  "term_id": "GO:0030674",
  "gene_name": "SH3 domain-binding glutamic acid-rich-like protein 2",
  "gene": "UniProtKB:Q9UJC5",
  "term_label": "protein-macromolecule adaptor activity"
}